BIR domain binding [GO:1990525] (molecular function) Definition: Binding to a Baculovirus Inhibitor of apoptosis protein Repeat (BIR) domain. Also known as: Baculovirus Inhibitor of apoptosis protein Repeat domain binding Sources: GOC:ha, InterPro:IPR001370 Note: An example of this is the Drosophila reaper gene in PMID:21886178. Relationships: is a type of protein domain specific binding [GO:0019904]